regulation of jasmonic acid mediated signaling pathway [GO:2000022] (biological process) Definition: Any process that modulates the frequency, rate or extent of jasmonic acid mediated signaling pathway. Sources: GOC:obol Also known as: regulation of jasmonic acid mediated signalling pathway Relationships: is a type of regulation of signal transduction [GO:0009966]; regulates jasmonic acid mediated signaling pathway [GO:0009867]